{
  "gene_symbol": "CCL15",
  "gene_name": "C-C motif chemokine 15",
  "term_id": "GO:0030335",
  "gene": "UniProtKB:Q16663",
  "term_label": "positive regulation of cell migration"
}